regulation of cell size [GO:0008361] (biological process) Also known as: cell size control Sources: GOC:go_curators Relationships: is a type of regulation of cellular component size [GO:0032535] Subtypes: cell volume homeostasis [GO:0006884], regulation of follicle cell microvillus length [GO:0032533], negative regulation of cell size [GO:0045792], GO:0045793, regulation of cell diameter [GO:0060305] Definition: Any process that modulates the size of a cell.